{
  "gene_symbol": "SLC17A1",
  "gene_name": "Sodium-dependent phosphate transport protein 1",
  "gene": "UniProtKB:Q14916",
  "term_id": "GO:0044341",
  "term_label": "sodium-dependent phosphate transport"
}